L-altrarate dehydratase activity [GO:1990594] (molecular function) References: PMID:17649980 Also known as: L-talarate dehydratase activity Definition: Catalysis of the reaction: L-altrarate = 5-dehydro-4-deoxy-D-glucarate + H2O. Relationships: is a type of hydro-lyase activity [GO:0016836]